{
  "term_id": "GO:0000976",
  "gene": "UniProtKB:Q8TF20",
  "term_label": "transcription cis-regulatory region binding",
  "gene_symbol": "ZNF721",
  "gene_name": "Zinc finger protein 721"
}